{
  "gene": "UniProtKB:Q9NQM4",
  "term_id": "GO:0045505",
  "gene_name": "Dynein axonemal assembly factor 6",
  "term_label": "dynein intermediate chain binding",
  "gene_symbol": "DNAAF6"
}